{
  "gene_symbol": "FAM162A",
  "term_id": "GO:0071456",
  "gene_name": "Protein FAM162A",
  "term_label": "cellular response to hypoxia",
  "gene": "UniProtKB:Q96A26"
}